{
  "gene_symbol": "SLC4A2",
  "term_id": "GO:0016324",
  "gene_name": "Anion exchange protein 2",
  "term_label": "apical plasma membrane",
  "gene": "UniProtKB:P04920"
}